{
  "term_id": "GO:0003677",
  "gene": "UniProtKB:O14646",
  "gene_symbol": "CHD1",
  "term_label": "DNA binding",
  "gene_name": "Chromodomain-helicase-DNA-binding protein 1"
}